synaptic target attraction [GO:0016200] (biological process) Definition: The process in which a neuronal cell in a multicellular organism recognizes chemoattractant signals from, and grows towards, potential targets. Sources: GOC:mah, ISBN:0878932437 Relationships: is a type of positive chemotaxis [GO:0050918]; is part of GO:0008039